{
  "gene": "UniProtKB:Q70IA8",
  "gene_name": "MOB kinase activator 3C",
  "term_label": "cytoplasm",
  "gene_symbol": "MOB3C",
  "term_id": "GO:0005737"
}